{
  "term_id": "UNKNOWN:0003",
  "gene_name": "Uncharacterized protein ZNF22-AS1",
  "gene_symbol": "ZNF22-AS1",
  "gene": "UniProtKB:Q5T742",
  "term_label": "Unknown cellular component"
}